{
  "gene_name": "OTU domain-containing protein 5",
  "term_label": "Unknown cellular component",
  "gene_symbol": "OTUD5",
  "term_id": "UNKNOWN:0003",
  "gene": "UniProtKB:Q96G74"
}